cell-cell adhesion mediated by cadherin [GO:0044331] (biological process) Regulation: regulated by regulation of cell-cell adhesion mediated by cadherin [GO:2000047]; negatively regulated by negative regulation of cell-cell adhesion mediated by cadherin [GO:2000048]; RO_0002213 by GO:2000049 Relationships: is a type of cell-cell adhesion [GO:0098609] References: PMID:10923970 Sources: GOC:ha, GOC:hjd, GOC:jl Definition: The attachment of one cell to another cell via a cadherin, transmembrane proteins having repeating extracellular calcium ion binding domains.